detection of electrical stimulus involved in sensory perception [GO:0050963] (biological process) Definition: The series of events in which an electrical stimulus is received by a cell and converted into a molecular signal as part of sensory perception. Relationships: is a type of GO:0050906; is_a detection of electrical stimulus [GO:0050981]; is part of sensory perception of electrical stimulus [GO:0050952] Sources: GOC:ai, GOC:dos Subtypes: GO:0050964, detection of electrical stimulus involved in sensory perception of pain [GO:0050967], GO:0050970 Also known as: sensory detection of electrical stimulus, sensory detection of electrical stimulus during sensory perception, sensory perception, sensory detection of electrical stimulus, sensory perception, sensory transduction of electrical stimulus, sensory transduction of electrical stimulus, sensory transduction of electrical stimulus during sensory perception